{
  "gene": "UniProtKB:Q07973",
  "term_id": "GO:0033280",
  "gene_symbol": "CYP24A1",
  "term_label": "response to vitamin D",
  "gene_name": "1,25-dihydroxyvitamin D(3) 24-hydroxylase, mitochondrial"
}